{
  "gene_symbol": "KRTAP19-3",
  "gene_name": "Keratin-associated protein 19-3",
  "gene": "UniProtKB:Q7Z4W3",
  "term_label": "Unknown molecular function",
  "term_id": "UNKNOWN:0001"
}